{
  "term_label": "membrane",
  "gene_symbol": "MAL",
  "gene": "UniProtKB:P21145",
  "gene_name": "Myelin and lymphocyte protein",
  "term_id": "GO:0016020"
}